{
  "gene": "UniProtKB:Q8TBZ3",
  "gene_name": "WD repeat-containing protein 20",
  "term_label": "cytoplasm",
  "gene_symbol": "WDR20",
  "term_id": "GO:0005737"
}